negative regulation of DNA-templated transcription, elongation [GO:0032785] (biological process) Sources: GOC:mah, GOC:txnOH Relationships: is a type of GO:0032784; is a type of negative regulation of DNA-templated transcription [GO:0045892]; negatively regulates GO:0006354 Also known as: down regulation of RNA elongation, down-regulation of RNA elongation, downregulation of RNA elongation, inhibition of RNA elongation, negative regulation of transcription elongation, negative regulation of transcriptional elongation, negative regulation of DNA-dependent transcription, elongation, negative regulation of transcription elongation, DNA-dependent, negative transcription elongation regulator activity Subtypes: GO:0034244, negative regulation of transcription elongation by RNA polymerase I [GO:2001208] Definition: Any process that stops, prevents, or reduces the frequency, rate or extent of transcription elongation, the extension of an RNA molecule after transcription initiation and promoter clearance by the addition of ribonucleotides catalyzed by a DNA-dependent RNA polymerase.